regulation of heptasaccharide transport [GO:1900294] (biological process) Sources: GOC:TermGenie, GOC:mengo_curators Definition: Any process that modulates the frequency, rate or extent of heptasaccharide transport. Subtypes: negative regulation of heptasaccharide transport [GO:1900295], positive regulation of heptasaccharide transport [GO:1900296], regulation of maltoheptaose transport [GO:1900306] Relationships: is a type of GO:0051049; regulates heptasaccharide transport [GO:2001104]